4,5-9,10-diseco-3-hydroxy-5,9,17-trioxoandrosta-1(10),2-diene-4-oate hydrolase activity [GO:0102296] (MF) Sources: GOC:pz, RHEA:32035 Definition: Catalysis of the reaction: (1E,2Z)-3-hydroxy-5,9,17-trioxo-4,5:9,10-disecoandrosta-1(10),2-dien-4-oate + H2O = 9,17-dioxo-1,2,3,4,10,19-hexanorandrostan-5-oate + (2Z,4Z)-2-hydroxyhexa-2,4-dienoate + H+. Relationships: is a type of hydrolase activity, acting on acid carbon-carbon bonds, in ketonic substances [GO:0016823]